antigen processing and presentation of endogenous peptide antigen via MHC class I via endolysosomal pathway [GO:0002487] (biological process) References: PMID:10631943 Sources: GOC:add Also known as: endogenous peptide antigen processing and presentation via MHC class I via endolysosomal pathway Relationships: is a type of antigen processing and presentation of endogenous peptide antigen via MHC class I [GO:0019885] Definition: The process in which an antigen-presenting cell expresses a peptide antigen of endogenous origin on its cell surface in association with an MHC class I protein complex. The peptide is typically a fragment of a larger endogenous protein which has been degraded within the cell and becomes associated with the MHC class I molecule in an endolysosome. Class I here refers to classical class I molecules.